{
  "gene_symbol": "CELA3A",
  "term_label": "extracellular space",
  "gene_name": "Chymotrypsin-like elastase family member 3A",
  "gene": "UniProtKB:P09093",
  "term_id": "GO:0005615"
}